purine nucleobase biosynthetic process [GO:0009113] (biological process) Subtypes: purine nucleobase salvage [GO:0043096], GO:0046084, guanine biosynthetic process [GO:0046099], GO:0046101, xanthine biosynthetic process [GO:0046111] Relationships: is_a purine nucleobase metabolic process [GO:0006144]; is a type of nucleobase biosynthetic process [GO:0046112]; is a type of GO:0072522 Also known as: purine base anabolism, purine base biosynthesis, purine base biosynthetic process, purine base formation, purine base synthesis Sources: ISBN:0198506732 Definition: The chemical reactions and pathways resulting in the formation of purine nucleobases, one of the two classes of nitrogen-containing ring compounds found in DNA and RNA, which include adenine and guanine.